{
  "term_id": "GO:0005886",
  "term_label": "plasma membrane",
  "gene_symbol": "REM1",
  "gene_name": "GTP-binding protein REM 1",
  "gene": "UniProtKB:O75628"
}